{
  "gene_symbol": "PRH2",
  "gene_name": "Salivary acidic proline-rich phosphoprotein 1_2",
  "gene": "UniProtKB:P02810",
  "term_label": "Unknown biological process",
  "term_id": "UNKNOWN:0002"
}